{
  "term_id": "GO:0009931",
  "term_label": "calcium-dependent protein serine/threonine kinase activity",
  "gene": "UniProtKB:Q8IW41",
  "gene_name": "MAP kinase-activated protein kinase 5",
  "gene_symbol": "MAPKAPK5"
}